{
  "term_label": "endosome",
  "gene": "UniProtKB:O43493",
  "gene_name": "Trans-Golgi network integral membrane protein 2",
  "gene_symbol": "TGOLN2",
  "term_id": "GO:0005768"
}